{
  "gene": "UniProtKB:Q14314",
  "term_id": "UNKNOWN:0001",
  "term_label": "Unknown molecular function",
  "gene_symbol": "FGL2",
  "gene_name": "Fibroleukin"
}